negative regulation of transcription by RNA polymerase II [GO:0000122] (biological process) Subtypes: carbon catabolite repression of transcription from RNA polymerase II promoter [GO:0000437], negative regulation of ribosomal protein gene transcription by RNA polymerase II [GO:0010688], negative regulation of transcription initiation by RNA polymerase II [GO:0060633], GO:0120191, negative regulation of snRNA transcription by RNA polymerase II [GO:1905381] Also known as: down regulation of transcription from RNA polymerase II promoter, down-regulation of transcription from RNA polymerase II promoter, downregulation of transcription from RNA polymerase II promoter, inhibition of transcription from RNA polymerase II promoter, negative regulation of transcription from Pol II promoter, negative regulation of transcription from RNA polymerase II promoter, down regulation of global transcription from RNA polymerase II promoter, down-regulation of global transcription from RNA polymerase II promoter, downregulation of global transcription from RNA polymerase II promoter, inhibition of global transcription from RNA polymerase II promoter, negative regulation of gene-specific transcription from RNA polymerase II promoter, negative regulation of global transcription from Pol II promoter, negative regulation of transcription from RNA polymerase II promoter, global Sources: GOC:go_curators, GOC:txnOH Relationships: is a type of GO:0006357; is a type of GO:0045892; negatively regulates transcription by RNA polymerase II [GO:0006366] Definition: Any process that stops, prevents, or reduces the frequency, rate or extent of transcription mediated by RNA polymerase II.